{
  "gene_symbol": "USHBP1",
  "term_id": "UNKNOWN:0002",
  "gene": "UniProtKB:Q8N6Y0",
  "gene_name": "Harmonin-binding protein USHBP1",
  "term_label": "Unknown biological process"
}